imaginal disc-derived wing hair organization [GO:0035317] (biological process) Note: See also the fly_anatomy.ontology term 'wing hair ; FBbt:00004340'. Definition: A process that is carried out at the cellular level that results in the assembly, arrangement of constituent parts, or disassembly of an imaginal disc-derived wing hair. A wing hair is an actin-rich, polarized, non-sensory apical projection that protrudes from each of the approximately 30,000 wing epithelial cells. An example of this is found in Drosophila melanogaster. Relationships: is a type of non-sensory hair organization [GO:0035316]; is part of GO:0007476 Also known as: wing hair organisation, wing trichome organization and biogenesis, imaginal disc-derived wing hair organization and biogenesis, wing hair organization and biogenesis References: PMID:11064425, PMID:12540853 Sources: GOC:mtg_sensu